{
  "gene_name": "Olfactory receptor 7A10",
  "term_id": "GO:0007165",
  "gene_symbol": "OR7A10",
  "gene": "UniProtKB:O76100",
  "term_label": "signal transduction"
}